positive regulation of NF-kappaB transcription factor activity [GO:0051092] (biological process) Also known as: NF-kappaB activation, activation of NF-kappaB, activation of NF-kappaB transcription factor Definition: Any process that activates or increases the frequency, rate or extent of activity of the transcription factor NF-kappaB. References: PMID:15087454, PMID:15170030 Sources: GOC:dph, GOC:tb Relationships: is a type of positive regulation of DNA-binding transcription factor activity [GO:0051091]